{
  "gene": "UniProtKB:P16050",
  "term_id": "GO:0050473",
  "gene_symbol": "ALOX15",
  "term_label": "arachidonate 15-lipoxygenase activity",
  "gene_name": "Polyunsaturated fatty acid lipoxygenase ALOX15"
}